{
  "gene_symbol": "IL12A",
  "term_id": "GO:0043514",
  "term_label": "interleukin-12 complex",
  "gene_name": "Interleukin-12 subunit alpha",
  "gene": "UniProtKB:P29459"
}